{
  "gene_name": "Nephrocystin-1",
  "gene_symbol": "NPHP1",
  "term_label": "Unknown molecular function",
  "term_id": "UNKNOWN:0001",
  "gene": "UniProtKB:O15259"
}